{
  "gene_name": "Myelin basic protein",
  "term_label": "myelination",
  "gene": "UniProtKB:P02686",
  "term_id": "GO:0042552",
  "gene_symbol": "MBP"
}